{
  "term_label": "Unknown cellular component",
  "gene_symbol": "PRR23E",
  "gene_name": "Proline-rich protein 23E",
  "gene": "UniProtKB:Q8N813",
  "term_id": "UNKNOWN:0003"
}